bacterial-type flagellum basal body, distal rod, L ring [GO:0009427] (cellular component) References: PMID:10572114, PMID:12624192 Sources: GOC:cilia, GOC:mtg_sensu Also known as: flagellar basal body, distal rod, L ring, flagellin-based flagellum basal body, distal rod, L ring Relationships: is a type of GO:0110165; is part of bacterial-type flagellum basal body, distal rod [GO:0009426] Definition: One of the rings of the bacterial-type flagellar basal body; anchors the basal body to the outer membrane.